non-collagenous component of basement membrane [GO:0140144] (cellular component) Relationships: is a type of external encapsulating structure [GO:0030312]; is part of solid phase of basement membrane [GO:0140139] Definition: The non-collagenous compartment of the solid phase in basement membrane ECM, including glycoproteins like laminins or nidogens. References: PMID:21421915, PMID:28324731